{
  "term_label": "cytosol",
  "term_id": "GO:0005829",
  "gene_symbol": "EIF2AK4",
  "gene": "UniProtKB:Q9P2K8",
  "gene_name": "eIF-2-alpha kinase GCN2"
}